M phase [GO:0000279] (BP) Subtypes: mitotic M phase [GO:0000087], meiotic M phase [GO:0051327] Definition: A cell cycle phase during which nuclear division occurs, and which is comprises the phases: prophase, metaphase, anaphase and telophase. Relationships: is a type of cell cycle phase [GO:0022403] Also known as: M-phase Sources: GOC:mtg_cell_cycle Note: Note that this term should not be used for direct annotation. If you are trying to make an annotation to x phase, it is likely that the correct annotation is 'regulation of x/y phase transition' or to a process which occurs during the reported phase (i.e mitotic DNA replication for mitotic S-phase). To capture the phase when a specific location or process is observed, the phase term can be used in an annotation extension (PMID:24885854) applied to a cellular component term (with the relation exists_during) or a biological process term (with the relation happens_during).